{
  "gene_symbol": "GFER",
  "term_id": "GO:0016971",
  "gene": "UniProtKB:P55789",
  "term_label": "flavin-dependent sulfhydryl oxidase activity",
  "gene_name": "FAD-linked sulfhydryl oxidase ALR"
}